DNA catabolic process [GO:0006308] (biological process) Subtypes: GO:0006309, mitochondrial DNA catabolic process [GO:0032043] Regulation: regulated by GO:1903624; negatively regulated by negative regulation of DNA catabolic process [GO:1903625]; positively regulated by GO:1903626 Also known as: DNA breakdown, DNA catabolism, DNA degradation Relationships: is a type of DNA metabolic process [GO:0006259]; is a type of nucleic acid catabolic process [GO:0141188]; has part DNA nuclease activity [GO:0004536] Sources: GOC:go_curators, ISBN:0198506732 Definition: The cellular DNA metabolic process resulting in the breakdown of DNA, deoxyribonucleic acid, one of the two main types of nucleic acid, consisting of a long unbranched macromolecule formed from one or two strands of linked deoxyribonucleotides, the 3'-phosphate group of each constituent deoxyribonucleotide being joined in 3',5'-phosphodiester linkage to the 5'-hydroxyl group of the deoxyribose moiety of the next one.